{
  "term_id": "GO:0060828",
  "gene": "UniProtKB:Q8N7R7",
  "gene_name": "Cyclin-Y-like protein 1",
  "term_label": "regulation of canonical Wnt signaling pathway",
  "gene_symbol": "CCNYL1"
}